{
  "gene": "UniProtKB:O14610",
  "gene_name": "Guanine nucleotide-binding protein G(I)_G(S)_G(O) subunit gamma-T2",
  "term_id": "GO:0031681",
  "term_label": "G-protein beta-subunit binding",
  "gene_symbol": "GNGT2"
}